{
  "gene_symbol": "Q8TCH9",
  "term_id": "UNKNOWN:0002",
  "term_label": "Unknown biological process",
  "gene": "UniProtKB:Q8TCH9",
  "gene_name": "Putative uncharacterized protein FLJ23865"
}